{
  "gene_symbol": "EDNRB",
  "gene": "UniProtKB:P24530",
  "gene_name": "Endothelin receptor type B",
  "term_id": "GO:0042310",
  "term_label": "vasoconstriction"
}